{
  "term_id": "GO:0003723",
  "gene_symbol": "EXOSC6",
  "term_label": "RNA binding",
  "gene": "UniProtKB:Q5RKV6",
  "gene_name": "Exosome complex component MTR3"
}